{
  "gene": "UniProtKB:P50221",
  "gene_symbol": "MEOX1",
  "term_id": "GO:0006357",
  "gene_name": "Homeobox protein MOX-1",
  "term_label": "regulation of transcription by RNA polymerase II"
}